{
  "gene_name": "Proline-rich protein 15",
  "term_label": "Unknown biological process",
  "term_id": "UNKNOWN:0002",
  "gene_symbol": "PRR15",
  "gene": "UniProtKB:Q8IV56"
}